anterograde axonal transport [GO:0008089] (biological process) Relationships: is a type of axonal transport [GO:0098930]; occurs in GO:1904115 Definition: The directed movement of organelles or molecules along microtubules from the cell body toward the cell periphery in nerve cell axons. Also known as: anterograde axon cargo transport Subtypes: GO:0048490, GO:0098957, GO:0099087, anterograde axonal protein transport [GO:0099641], anterograde neuronal dense core vesicle transport [GO:1990048] Sources: ISBN:0815316194